{
  "gene": "UniProtKB:A0A096LP01",
  "term_label": "Unknown biological process",
  "gene_symbol": "SMIM26",
  "gene_name": "Small integral membrane protein 26",
  "term_id": "UNKNOWN:0002"
}